{
  "gene": "UniProtKB:Q6P1K8",
  "term_id": "GO:0006357",
  "gene_symbol": "GTF2H2C",
  "gene_name": "General transcription factor IIH subunit 2-like protein",
  "term_label": "regulation of transcription by RNA polymerase II"
}